{
  "gene": "UniProtKB:Q5VT97",
  "term_id": "GO:0016477",
  "gene_symbol": "SYDE2",
  "gene_name": "Rho GTPase-activating protein SYDE2",
  "term_label": "cell migration"
}